{
  "gene_name": "Short stature homeobox protein 2",
  "gene_symbol": "SHOX2",
  "gene": "UniProtKB:O60902",
  "term_label": "regulation of transcription by RNA polymerase II",
  "term_id": "GO:0006357"
}